{
  "gene_symbol": "ZNF70",
  "term_id": "GO:0000977",
  "gene": "UniProtKB:Q9UC06",
  "gene_name": "Zinc finger protein 70",
  "term_label": "RNA polymerase II transcription regulatory region sequence-specific DNA binding"
}